hyphae septin collar [GO:0062140] (cellular component) Relationships: is_a septin collar [GO:0032173] Also known as: septin collar of invasive hyphae References: PMID:29567712 Definition: A septin collar in pathogenic fungi involved in the constriction of hyphae at the plant plasmodesma enabling penetration of an adjacent cell.